{
  "gene_name": "Reticulon-3",
  "term_label": "neuron projection",
  "gene": "UniProtKB:O95197",
  "gene_symbol": "RTN3",
  "term_id": "GO:0043005"
}